{
  "gene_name": "Protein SEC13 homolog",
  "term_id": "GO:0090114",
  "term_label": "COPII-coated vesicle budding",
  "gene_symbol": "SEC13",
  "gene": "UniProtKB:P55735"
}